{
  "term_label": "extracellular matrix",
  "gene": "UniProtKB:Q9NS15",
  "gene_symbol": "LTBP3",
  "term_id": "GO:0031012",
  "gene_name": "Latent-transforming growth factor beta-binding protein 3"
}